regulation of cell proliferation involved in heart valve morphogenesis [GO:0003250] (biological process) Sources: GOC:mtg_heart Subtypes: positive regulation of cell proliferation involved in heart valve morphogenesis [GO:0003251], GO:0003252 Relationships: is a type of GO:2000136; RO_0002211 cell proliferation involved in heart valve morphogenesis [GO:0003249] Definition: Any process that modulates the rate, frequency or extent of cell proliferation that contributes to the shaping of a heart valve.